{
  "gene_name": "Arginine and glutamate-rich protein 1",
  "term_label": "nucleoplasm",
  "gene": "UniProtKB:Q9NWB6",
  "gene_symbol": "ARGLU1",
  "term_id": "GO:0005654"
}